{
  "term_label": "serine-type endopeptidase activity",
  "term_id": "GO:0004252",
  "gene": "UniProtKB:P07288",
  "gene_name": "Prostate-specific antigen",
  "gene_symbol": "KLK3"
}